{
  "term_id": "GO:0005525",
  "gene_symbol": "GBP3",
  "term_label": "GTP binding",
  "gene": "UniProtKB:Q9H0R5",
  "gene_name": "Guanylate-binding protein 3"
}